{
  "term_id": "UNKNOWN:0001",
  "gene_name": "Radial spoke head 14 homolog",
  "gene_symbol": "RSPH14",
  "gene": "UniProtKB:Q9UHP6",
  "term_label": "Unknown molecular function"
}